{
  "gene_symbol": "TADA2B",
  "gene_name": "Transcriptional adapter 2-beta",
  "gene": "UniProtKB:Q86TJ2",
  "term_id": "GO:0070461",
  "term_label": "SAGA-type complex"
}